{
  "term_label": "regulation of Rho protein signal transduction",
  "term_id": "GO:0035023",
  "gene_symbol": "ARHGEF18",
  "gene_name": "Rho guanine nucleotide exchange factor 18",
  "gene": "UniProtKB:Q6ZSZ5"
}